{
  "term_label": "extracellular space",
  "gene_symbol": "AMH",
  "term_id": "GO:0005615",
  "gene": "UniProtKB:P03971",
  "gene_name": "Muellerian-inhibiting factor"
}